{
  "gene_name": "M-phase inducer phosphatase 3",
  "gene": "UniProtKB:P30307",
  "gene_symbol": "CDC25C",
  "term_id": "GO:0005634",
  "term_label": "nucleus"
}